{
  "term_label": "tetrahydrofolate metabolic process",
  "gene": "UniProtKB:P34896",
  "gene_symbol": "SHMT1",
  "term_id": "GO:0046653",
  "gene_name": "Serine hydroxymethyltransferase, cytosolic"
}